{
  "term_id": "GO:0042797",
  "gene_symbol": "POLR2E",
  "gene": "UniProtKB:P19388",
  "term_label": "tRNA transcription by RNA polymerase III",
  "gene_name": "DNA-directed RNA polymerases I, II, and III subunit RPABC1"
}